{
  "gene_symbol": "PLPP4",
  "gene_name": "Phospholipid phosphatase 4",
  "gene": "UniProtKB:Q5VZY2",
  "term_label": "phospholipid metabolic process",
  "term_id": "GO:0006644"
}